{
  "gene": "UniProtKB:Q96PN7",
  "gene_symbol": "TRERF1",
  "term_id": "GO:0006357",
  "gene_name": "Transcriptional-regulating factor 1",
  "term_label": "regulation of transcription by RNA polymerase II"
}